{
  "term_id": "GO:0043410",
  "gene_name": "Fibroblast growth factor 16",
  "gene": "UniProtKB:O43320",
  "term_label": "positive regulation of MAPK cascade",
  "gene_symbol": "FGF16"
}